{
  "gene": "UniProtKB:Q13591",
  "term_label": "axon extension",
  "gene_symbol": "SEMA5A",
  "gene_name": "Semaphorin-5A",
  "term_id": "GO:0048675"
}